{
  "term_label": "Unknown biological process",
  "gene_symbol": "FAM90A2P",
  "gene_name": "Putative protein FAM90A2P",
  "gene": "UniProtKB:Q658T7",
  "term_id": "UNKNOWN:0002"
}